thymus development [GO:0048538] (biological process) Definition: The process whose specific outcome is the progression of the thymus over time, from its formation to the mature structure. The thymus is a symmetric bi-lobed organ involved primarily in the differentiation of immature to mature T cells, with unique vascular, nervous, epithelial, and lymphoid cell components. Relationships: is a type of GO:0048534; is a type of gland development [GO:0048732] Note: Note that this term is reserved for annotation of gene products involved in the formation of the thymus itself, not for gene products involved in T cell differentiation in the thymus or elsewhere. Sources: GOC:add, ISBN:0781735149